(1->3)-beta-D-glucan immune receptor activity [GO:0001874] (molecular function) Definition: Combining with (1->3)-beta-D-glucans to initiate an innate immune response. Also known as: (1->3)-beta-D-glucan receptor activity, (1,3)-beta-D-glucan receptor activity, 1,3-beta-D-glucan receptor activity, beta-1,3-D-glucan receptor activity, zymosan receptor activity Relationships: is a type of polysaccharide immune receptor activity [GO:0001873]; has part (1->3)-beta-D-glucan binding [GO:0001872] References: PMID:14707091